{
  "gene_symbol": "GPRC5C",
  "gene": "UniProtKB:Q9NQ84",
  "term_id": "UNKNOWN:0002",
  "gene_name": "G-protein coupled receptor family C group 5 member C",
  "term_label": "Unknown biological process"
}